{
  "gene_name": "Insulin-degrading enzyme",
  "gene": "UniProtKB:P14735",
  "gene_symbol": "IDE",
  "term_id": "GO:1901143",
  "term_label": "insulin catabolic process"
}